{
  "term_label": "cell surface receptor protein tyrosine kinase signaling pathway",
  "gene_symbol": "DOK5",
  "term_id": "GO:0007169",
  "gene_name": "Docking protein 5",
  "gene": "UniProtKB:Q9P104"
}